{
  "term_label": "calcium-dependent protein binding",
  "gene_symbol": "S100A1",
  "term_id": "GO:0048306",
  "gene_name": "Protein S100-A1",
  "gene": "UniProtKB:P23297"
}